{
  "gene_symbol": "BMPR2",
  "term_id": "GO:0071363",
  "gene": "UniProtKB:Q13873",
  "gene_name": "Bone morphogenetic protein receptor type-2",
  "term_label": "cellular response to growth factor stimulus"
}